triglyceride-sterol O-acyltransferase activity [GO:0047197] (molecular function) Also known as: triacylglycerol-sterol O-acyltransferase activity, triacylglycerol:3beta-hydroxysterol O-acyltransferase activity, triacylglycerol:sterol acyltransferase activity Definition: Catalysis of the reaction: a 3-beta-hydroxysterol + triacylglycerol = a 3-beta-hydroxysterol ester + 1,2-diacylglycerol. Relationships: is a type of O-acyltransferase activity [GO:0008374] Sources: EC:2.3.1.77, MetaCyc:2.3.1.77-RXN